{
  "gene_name": "Agouti-related protein",
  "term_id": "GO:0008343",
  "gene": "UniProtKB:O00253",
  "term_label": "adult feeding behavior",
  "gene_symbol": "AGRP"
}